dauer exit [GO:0043054] (biological process) Definition: Exit from the facultative diapause of the dauer (enduring) larval stage of nematode development. References: PMID:12620986 Sources: GOC:cab1 Relationships: is_a exit from diapause [GO:0071981]; is part of dauer larval development [GO:0040024] Also known as: exit from nematode dormancy